{
  "gene": "UniProtKB:Q16589",
  "term_label": "nucleus",
  "term_id": "GO:0005634",
  "gene_name": "Cyclin-G2",
  "gene_symbol": "CCNG2"
}